{
  "term_id": "GO:0004879",
  "term_label": "nuclear receptor activity",
  "gene": "UniProtKB:Q03181",
  "gene_name": "Peroxisome proliferator-activated receptor delta",
  "gene_symbol": "PPARD"
}